{
  "gene_name": "Putative annexin A2-like protein",
  "term_label": "positive regulation of plasminogen activation",
  "gene": "UniProtKB:A6NMY6",
  "gene_symbol": "ANXA2P2",
  "term_id": "GO:0010756"
}